BRCA1-B complex [GO:0070532] (cellular component) References: PMID:16391231 Sources: GOC:mah Relationships: is a type of nuclear protein-containing complex [GO:0140513] Definition: A protein complex that contains the BRCA1-BARD1 heterodimer, BACH1 and TopBP1, and binds to DNA during S phase at DNA damage sites.